{
  "term_id": "GO:0035556",
  "gene_name": "Serine_threonine-protein kinase ICK",
  "term_label": "intracellular signal transduction",
  "gene": "UniProtKB:Q9UPZ9",
  "gene_symbol": "CILK1"
}